selenite:proton symporter activity [GO:0097079] (molecular function) Definition: Enables the transfer of a solute or solutes from one side of a membrane to the other according to the reaction: selenite(out) + H+(out) = selenite(in) + H+(in). Relationships: is a type of solute:proton symporter activity [GO:0015295] Also known as: selenite:H+ symporter activity, selenite:hydrogen symporter activity References: PMID:20861301 Sources: GOC:mcc